{
  "gene": "UniProtKB:Q96P31",
  "gene_name": "Fc receptor-like protein 3",
  "gene_symbol": "FCRL3",
  "term_id": "GO:0009897",
  "term_label": "external side of plasma membrane"
}